positive regulation of juvenile hormone secretion [GO:0045973] (biological process) Sources: GOC:go_curators Also known as: up regulation of juvenile hormone secretion, up-regulation of juvenile hormone secretion, upregulation of juvenile hormone secretion, activation of juvenile hormone secretion, stimulation of juvenile hormone secretion Definition: Any process that activates or increases the frequency, rate or extent of the regulated release of juvenile hormone. Relationships: is a type of regulation of juvenile hormone secretion [GO:0007558]; is a type of positive regulation of lipid transport [GO:0032370]; is a type of GO:0046887; RO_0002213 juvenile hormone secretion [GO:0045443]